{
  "gene": "UniProtKB:O75112",
  "gene_symbol": "LDB3",
  "term_label": "muscle alpha-actinin binding",
  "gene_name": "LIM domain-binding protein 3",
  "term_id": "GO:0051371"
}